2-oxobutyrate biosynthetic process [GO:0046360] (biological process) Also known as: 2-oxobutyrate anabolism, 2-oxobutyrate biosynthesis, 2-oxobutyrate formation, 2-oxobutyrate synthesis, alpha-ketobutyrate biosynthesis, alpha-ketobutyrate biosynthetic process Definition: The chemical reactions and pathways resulting in the formation of 2-oxobutyrate, the anion of the organic acid 2-oxobutyric acid, which contains a ketone group on carbon 2. Relationships: is a type of short-chain fatty acid biosynthetic process [GO:0051790] Sources: ISBN:0198506732